{
  "gene": "UniProtKB:Q9UHI7",
  "gene_name": "Solute carrier family 23 member 1",
  "term_label": "Unknown biological process",
  "term_id": "UNKNOWN:0002",
  "gene_symbol": "SLC23A1"
}